{
  "gene_symbol": "IQGAP1",
  "gene_name": "Ras GTPase-activating-like protein IQGAP1",
  "term_id": "GO:0051015",
  "term_label": "actin filament binding",
  "gene": "UniProtKB:P46940"
}